negative regulation of glucomannan catabolic process [GO:2000907] (biological process) Definition: Any process that stops, prevents or reduces the frequency, rate or extent of glucomannan catabolic process. Sources: GOC:mengo_curators Also known as: negative regulation of glucomannan catabolism Relationships: is a type of negative regulation of catabolic process [GO:0009895]; is a type of negative regulation of macromolecule metabolic process [GO:0010605]; is a type of GO:0045912; is_a regulation of glucomannan catabolic process [GO:2000898]; negatively regulates glucomannan catabolic process [GO:2000884]